{
  "gene_symbol": "ID2",
  "term_id": "GO:0030182",
  "gene_name": "DNA-binding protein inhibitor ID-2",
  "gene": "UniProtKB:Q02363",
  "term_label": "neuron differentiation"
}